{
  "term_id": "GO:0004930",
  "gene_name": "Neuropeptide FF receptor 2",
  "gene": "UniProtKB:Q9Y5X5",
  "gene_symbol": "NPFFR2",
  "term_label": "G protein-coupled receptor activity"
}